{
  "term_label": "signal transduction",
  "term_id": "GO:0007165",
  "gene_name": "Putative olfactory receptor 1F2",
  "gene": "UniProtKB:Q96R84",
  "gene_symbol": "OR1F2P"
}